{
  "term_id": "GO:0005737",
  "gene": "UniProtKB:Q9UQ16",
  "term_label": "cytoplasm",
  "gene_name": "Dynamin-3",
  "gene_symbol": "DNM3"
}